{
  "gene_symbol": "GLS",
  "term_id": "UNKNOWN:0003",
  "gene": "UniProtKB:O94925",
  "gene_name": "Glutaminase kidney isoform, mitochondrial",
  "term_label": "Unknown cellular component"
}